{
  "gene_symbol": "HOXC9",
  "term_id": "GO:0009952",
  "gene_name": "Homeobox protein Hox-C9",
  "gene": "UniProtKB:P31274",
  "term_label": "anterior/posterior pattern specification"
}